{
  "term_id": "GO:0046513",
  "gene": "UniProtKB:O15121",
  "term_label": "ceramide biosynthetic process",
  "gene_name": "Sphingolipid delta(4)-desaturase DES1",
  "gene_symbol": "DEGS1"
}